{
  "term_id": "GO:0000786",
  "gene": "UniProtKB:P0DPK2",
  "gene_name": "Histone H3.Y",
  "gene_symbol": "H3Y1",
  "term_label": "nucleosome"
}